{
  "gene_name": "Polycystin-2",
  "gene": "UniProtKB:Q13563",
  "gene_symbol": "PKD2",
  "term_id": "GO:0071805",
  "term_label": "potassium ion transmembrane transport"
}